{
  "term_label": "protein processing",
  "gene_name": "Transmembrane protease serine 11F",
  "term_id": "GO:0016485",
  "gene_symbol": "TMPRSS11F",
  "gene": "UniProtKB:Q6ZWK6"
}